{
  "gene": "UniProtKB:Q8NGE5",
  "gene_symbol": "OR10A7",
  "term_id": "GO:0004984",
  "gene_name": "Olfactory receptor 10A7",
  "term_label": "olfactory receptor activity"
}